ciliary pocket membrane [GO:0020018] (cellular component) Also known as: cilial pocket membrane, cilium pocket membrane, flagellar pocket membrane Sources: GOC:cilia, GOC:mb Note: Note that cilia and eukaryotic flagella are deemed to be equivalent. In this case community usage is mostly 'flagellar', but the primary term name reflects the cilium parentage. Relationships: is a type of ciliary membrane [GO:0060170]; is part of ciliary pocket [GO:0020016] Definition: That part of the plasma membrane found in the ciliary pocket (also called flagellar pocket).